positive regulation of transcription from RNA polymerase II promoter by galactose [GO:0000435] (biological process) Sources: GOC:krc Relationships: is_a positive regulation of transcription by galactose [GO:0000411]; is a type of regulation of transcription from RNA polymerase II promoter by galactose [GO:0000431]; is a type of carbon catabolite activation of transcription from RNA polymerase II promoter [GO:0000436] Also known as: up regulation of transcription from RNA polymerase II promoter by galactose, up-regulation of transcription from RNA polymerase II promoter by galactose, upregulation of transcription from RNA polymerase II promoter by galactose, activation of transcription from RNA polymerase II promoter by galactose, stimulation of transcription from RNA polymerase II promoter by galactose Definition: Any process involving galactose that activates or increases the rate of transcription from an RNA polymerase II promoter.